plant-type cell wall modification involved in stomatal movement [GO:1905588] (biological process) References: PMID:27720618 Sources: GOC:TermGenie, GO_REF:0000060 Relationships: is a type of plant-type cell wall modification [GO:0009827]; BFO_0000050 GO:0010118 Definition: Any plant-type cell wall modification that is involved in stomatal movement. Also known as: cellulose and pectin-containing cell wall modification involved in stomatal movement